{
  "gene_name": "DNA polymerase iota",
  "term_id": "GO:0019985",
  "term_label": "translesion synthesis",
  "gene": "UniProtKB:Q9UNA4",
  "gene_symbol": "POLI"
}